{
  "gene_name": "C1q-related factor",
  "term_label": "synapse",
  "term_id": "GO:0045202",
  "gene_symbol": "C1QL1",
  "gene": "UniProtKB:O75973"
}